{
  "term_id": "GO:0006357",
  "gene": "UniProtKB:Q01860",
  "term_label": "regulation of transcription by RNA polymerase II",
  "gene_symbol": "POU5F1",
  "gene_name": "POU domain, class 5, transcription factor 1"
}